carnosine synthase activity [GO:0047730] (molecular function) Definition: Catalysis of the reaction: beta-alanine + L-histidine + ATP = carnosine + ADP + phosphate + H+. Relationships: is a type of acid-amino acid ligase activity [GO:0016881] Also known as: L-histidine:beta-alanine ligase (AMP-forming), carnosine synthetase activity, carnosine-anserine synthetase activity, carnosine-homocarnosine synthetase activity, homocarnosine-carnosine synthetase activity Sources: RHEA:19297